{
  "term_id": "GO:0005886",
  "term_label": "plasma membrane",
  "gene_name": "Olfactory receptor 2A12",
  "gene": "UniProtKB:Q8NGT7",
  "gene_symbol": "OR2A12"
}